{
  "gene_name": "Isoleucine--tRNA ligase, cytoplasmic",
  "gene_symbol": "IARS1",
  "term_id": "UNKNOWN:0003",
  "gene": "UniProtKB:P41252",
  "term_label": "Unknown cellular component"
}